{
  "term_label": "positive regulation of cell migration",
  "gene_symbol": "SEMA3E",
  "gene_name": "Semaphorin-3E",
  "term_id": "GO:0030335",
  "gene": "UniProtKB:O15041"
}